{
  "term_label": "maturation of 5.8S rRNA",
  "gene_name": "Eukaryotic translation initiation factor 6",
  "gene_symbol": "EIF6",
  "gene": "UniProtKB:P56537",
  "term_id": "GO:0000460"
}